{
  "term_id": "GO:0061630",
  "gene_symbol": "UBE3C",
  "gene": "UniProtKB:Q15386",
  "term_label": "ubiquitin protein ligase activity",
  "gene_name": "Ubiquitin-protein ligase E3C"
}